renal absorption [GO:0070293] (BP) Also known as: nephron absorption, renal reabsorption Relationships: is a type of renal system process [GO:0003014] Subtypes: renal D-glucose absorption [GO:0035623], renal sodium ion absorption [GO:0070294], renal water absorption [GO:0070295], renal protein absorption [GO:0097017], GO:0097291, renal amino acid absorption [GO:1990297] Definition: A renal system process in which water, ions, glucose and proteins are taken up from the collecting ducts, glomerulus and proximal and distal loops of the nephron. In non-mammalian species, absorption may occur in related structures (e.g. protein absorption is observed in nephrocytes in Drosophila, see PMID:23264686). Sources: GOC:dph, GOC:mah, GOC:yaf